{
  "gene": "UniProtKB:O14511",
  "gene_symbol": "NRG2",
  "term_label": "extracellular space",
  "gene_name": "Pro-neuregulin-2, membrane-bound isoform",
  "term_id": "GO:0005615"
}